trans-synaptic signaling by soluble gas [GO:0099543] (biological process) Definition: Cell-cell signaling between presynapse and postsynapse mediated by a soluble gas ligand crossing the synaptic cleft. Relationships: is a type of trans-synaptic signaling [GO:0099537] Sources: GOC:dos Subtypes: retrograde trans-synaptic signaling by soluble gas [GO:0098923], trans-synaptic signaling by nitric oxide [GO:0099548], trans-synaptic signaling by carbon monoxide [GO:0099549], trans-synaptic signaling by soluble gas, modulating synaptic transmission [GO:0099554]